2 iron, 2 sulfur cluster binding [GO:0051537] (molecular function) References: PMID:15952888 Sources: GOC:ai, Wikipedia:Iron-sulfur_cluster Definition: Binding to a 2 iron, 2 sulfur (2Fe-2S) cluster; this cluster consists of two iron atoms, with two inorganic sulfur atoms found between the irons and acting as bridging ligands. Also known as: 2 Fe 2 S cluster binding, 2 iron, 2 sulphur cluster binding, 2Fe-2S cluster binding, diiron disulfide cluster binding, diiron disulphide cluster binding, iron-sulfur cluster 2Fe-2S binding, iron-sulphur cluster 2Fe-2S binding Relationships: is a type of iron-sulfur cluster binding [GO:0051536]